{
  "gene_name": "Sorting nexin-9",
  "term_label": "plasma membrane tubulation",
  "gene": "UniProtKB:Q9Y5X1",
  "term_id": "GO:0097320",
  "gene_symbol": "SNX9"
}